S-(hydroxymethyl)glutathione dehydrogenase (NADP+) activity [GO:0106321] (molecular function) Sources: RHEA:19981 Definition: Catalysis of the reaction: S-(hydroxymethyl)glutathione + NADP+ = S-formylglutathione + NADPH + H+. Relationships: is a type of S-(hydroxymethyl)glutathione dehydrogenase [NAD(P)+] activity [GO:0051903]